{
  "gene": "UniProtKB:Q13114",
  "term_id": "GO:0043122",
  "gene_name": "TNF receptor-associated factor 3",
  "term_label": "regulation of canonical NF-kappaB signal transduction",
  "gene_symbol": "TRAF3"
}